{
  "gene_symbol": "RAB38",
  "term_id": "GO:0005739",
  "term_label": "mitochondrion",
  "gene_name": "Ras-related protein Rab-38",
  "gene": "UniProtKB:P57729"
}